{
  "gene": "UniProtKB:Q16842",
  "term_id": "GO:0097503",
  "term_label": "sialylation",
  "gene_symbol": "ST3GAL2",
  "gene_name": "CMP-N-acetylneuraminate-beta-galactosamide-alpha-2,3-sialyltransferase 2"
}